{
  "gene_symbol": "HIVEP3",
  "term_label": "regulation of transcription by RNA polymerase II",
  "gene_name": "Transcription factor HIVEP3",
  "gene": "UniProtKB:Q5T1R4",
  "term_id": "GO:0006357"
}